{
  "gene_name": "Transcription activator BRG1",
  "gene_symbol": "SMARCA4",
  "gene": "UniProtKB:P51532",
  "term_label": "chromatin binding",
  "term_id": "GO:0003682"
}